{
  "term_id": "UNKNOWN:0001",
  "gene": "UniProtKB:A4QPH2",
  "term_label": "Unknown molecular function",
  "gene_symbol": "PI4KAP2",
  "gene_name": "Putative phosphatidylinositol 4-kinase alpha-like protein P2"
}